{
  "gene": "UniProtKB:Q9H6W3",
  "term_id": "GO:0032453",
  "term_label": "histone H3K4 demethylase activity",
  "gene_symbol": "RIOX1",
  "gene_name": "Ribosomal oxygenase 1"
}